{
  "gene": "UniProtKB:Q0JRZ9",
  "gene_symbol": "FCHO2",
  "term_id": "GO:0048488",
  "gene_name": "F-BAR domain only protein 2",
  "term_label": "synaptic vesicle endocytosis"
}